{
  "term_id": "GO:0002767",
  "gene": "UniProtKB:P59901",
  "term_label": "immune response-inhibiting cell surface receptor signaling pathway",
  "gene_name": "Leukocyte immunoglobulin-like receptor subfamily A member 4",
  "gene_symbol": "LILRA4"
}